{
  "term_label": "DNA-binding transcription factor activity, RNA polymerase II-specific",
  "gene": "UniProtKB:Q96N58",
  "gene_symbol": "ZNF578",
  "term_id": "GO:0000981",
  "gene_name": "Zinc finger protein 578"
}